{
  "gene_symbol": "GUCY1B1",
  "gene_name": "Guanylate cyclase soluble subunit beta-1",
  "gene": "UniProtKB:Q02153",
  "term_label": "response to oxygen levels",
  "term_id": "GO:0070482"
}